{
  "term_id": "GO:0006940",
  "term_label": "regulation of smooth muscle contraction",
  "gene_symbol": "CHRM2",
  "gene": "UniProtKB:P08172",
  "gene_name": "Muscarinic acetylcholine receptor M2"
}